{
  "gene_symbol": "TAAR8",
  "term_label": "trace-amine receptor activity",
  "gene_name": "Trace amine-associated receptor 8",
  "gene": "UniProtKB:Q969N4",
  "term_id": "GO:0001594"
}